{
  "gene": "UniProtKB:Q15052",
  "gene_name": "Rho guanine nucleotide exchange factor 6",
  "gene_symbol": "ARHGEF6",
  "term_label": "lamellipodium assembly",
  "term_id": "GO:0030032"
}